1-hydroxy-2-naphthoate 1,2-dioxygenase activity [GO:0018582] (molecular function) Definition: Catalysis of the reaction: 1-hydroxy-2-naphthoate + O2 = (3E)-4-(2-carboxyphenyl)-2-oxobut-3-enoate. Relationships: is a type of oxidoreductase activity, acting on single donors with incorporation of molecular oxygen, incorporation of two atoms of oxygen [GO:0016702] Sources: EC:1.13.11.38 Also known as: 1-hydroxy-2-naphthoate dioxygenase activity, 1-hydroxy-2-naphthoate-degrading enzyme activity, 1-hydroxy-2-naphthoate:oxygen 1,2-oxidoreductase (decyclizing), 1-hydroxy-2-naphthoic acid dioxygenase activity